detection of lipoteichoic acid [GO:0070392] (biological process) Definition: The series of events in which a lipoteichoic acid stimulus is received by a cell and converted into a molecular signal; lipoteichoic acid is a major component of the cell wall of gram-positive bacteria and typically consists of a chain of glycerol-phosphate repeating units linked to a glycolipid anchor. References: PMID:14665680, PMID:16020688 Sources: GOC:add Also known as: detection of LTA Relationships: is a type of GO:0032490; is a type of response to lipoteichoic acid [GO:0070391]